{
  "gene": "UniProtKB:Q8N3U4",
  "gene_name": "Cohesin subunit SA-2",
  "gene_symbol": "STAG2",
  "term_label": "chromatin",
  "term_id": "GO:0000785"
}